{
  "gene": "UniProtKB:Q6IEG0",
  "gene_name": "U11_U12 small nuclear ribonucleoprotein 48 kDa protein",
  "term_id": "UNKNOWN:0001",
  "term_label": "Unknown molecular function",
  "gene_symbol": "SNRNP48"
}